1-phosphatidyl-1D-myo-inositol 4,5-bisphosphate catabolic process [GO:1902634] (biological process) Relationships: is_a phosphatidylinositol catabolic process [GO:0031161]; is a type of 1-phosphatidyl-1D-myo-inositol 4,5-bisphosphate metabolic process [GO:1902633] Regulation: regulated by regulation of 1-phosphatidyl-1D-myo-inositol 4,5-bisphosphate catabolic process [GO:1902641]; negatively regulated by negative regulation of 1-phosphatidyl-1D-myo-inositol 4,5-bisphosphate catabolic process [GO:1902642]; RO_0002213 by GO:1902643 References: PMID:22562153 Sources: GOC:TermGenie, GOC:di, GO_REF:0000068 Definition: The chemical reactions and pathways resulting in the breakdown of 1-phosphatidyl-1D-myo-inositol 4,5-bisphosphate. Note: Phosphatidylinositol-4,5-bisphosphate, PtdIns(4,5)P(2) common name. Also known as: 1-phosphatidyl-1D-myo-inositol 4,5-bisphosphate breakdown, 1-phosphatidyl-1D-myo-inositol 4,5-bisphosphate catabolism, 1-phosphatidyl-1D-myo-inositol 4,5-bisphosphate degradation